{
  "gene_name": "Ropporin-1-like protein",
  "gene_symbol": "ROPN1L",
  "term_id": "GO:0030317",
  "gene": "UniProtKB:Q96C74",
  "term_label": "flagellated sperm motility"
}